{
  "gene_name": "BAG family molecular chaperone regulator 5",
  "term_id": "GO:0031397",
  "term_label": "negative regulation of protein ubiquitination",
  "gene_symbol": "BAG5",
  "gene": "UniProtKB:Q9UL15"
}